positive regulation of alpha-beta T cell proliferation [GO:0046641] (biological process) Also known as: positive regulation of alpha-beta T lymphocyte proliferation, positive regulation of alpha-beta T-cell proliferation, positive regulation of alpha-beta T-lymphocyte proliferation, up regulation of alpha-beta T cell proliferation, up-regulation of alpha-beta T cell proliferation, upregulation of alpha-beta T cell proliferation, activation of alpha-beta T cell proliferation, stimulation of alpha-beta T cell proliferation Relationships: is a type of positive regulation of T cell proliferation [GO:0042102]; is a type of positive regulation of alpha-beta T cell activation [GO:0046635]; is a type of regulation of alpha-beta T cell proliferation [GO:0046640]; positively regulates alpha-beta T cell proliferation [GO:0046633] Definition: Any process that activates or increases the frequency, rate or extent of alpha-beta T cell proliferation. Sources: GOC:ai Subtypes: positive regulation of NK T cell proliferation [GO:0051142], positive regulation of CD4-positive, alpha-beta T cell proliferation [GO:2000563], positive regulation of CD8-positive, alpha-beta T cell proliferation [GO:2000566]